versicolorin B desaturase activity [GO:0140398] (molecular function) Relationships: is a type of oxidoreductase activity, acting on paired donors, with oxidation of a pair of donors resulting in the reduction of molecular oxygen to two molecules of water [GO:0016717] References: PMID:15006741, PMID:8368837 Definition: Catalyzes the reaction: versicolorin B + NADPH + O2 = versicolorin A + NADP+ + 2 H2O. Uses heme-thiolate as a co-factor. Involved in the synthesis of aflatoxins in the fungus Aspergillus parasiticus.